{
  "term_id": "GO:0061630",
  "gene_name": "E3 ubiquitin-protein ligase TRIM21",
  "gene_symbol": "TRIM21",
  "term_label": "ubiquitin protein ligase activity",
  "gene": "UniProtKB:P19474"
}